{
  "term_id": "GO:0032880",
  "gene_symbol": "CAMK1",
  "gene": "UniProtKB:Q14012",
  "term_label": "regulation of protein localization",
  "gene_name": "Calcium_calmodulin-dependent protein kinase type 1"
}